{
  "gene_name": "AT-rich interactive domain-containing protein 1A",
  "gene_symbol": "ARID1A",
  "term_label": "positive regulation of DNA-templated transcription",
  "term_id": "GO:0045893",
  "gene": "UniProtKB:O14497"
}